{
  "gene_name": "Mitogen-activated protein kinase kinase kinase 8",
  "term_label": "Unknown cellular component",
  "gene": "UniProtKB:P41279",
  "term_id": "UNKNOWN:0003",
  "gene_symbol": "MAP3K8"
}